middle viral transcription [GO:0019084] (biological process) Sources: GOC:bf, GOC:jl Definition: The viral transcription that takes place after early transcription in the viral life cycle, and which involves the transcription of genes required for replication. Relationships: is a type of viral transcription [GO:0019083] Also known as: (delayed) early viral mRNA transcription